ribonuclease P RNA binding [GO:0033204] (MF) Definition: Binding to RNA subunit of ribonuclease P. References: PMID:11455963 Sources: GOC:pg Also known as: RNase P RNA binding Relationships: is a type of GO:0003723